laminin binding involved in cell-matrix adhesion [GO:0098638] (molecular function) Relationships: is a type of laminin binding [GO:0043236]; is a type of GO:0098634 Sources: GOC:dos Definition: Any laminin protein binding that occurs as part of cell-matrix adhesion.